{
  "gene_symbol": "LLGL1",
  "gene_name": "Lethal(2) giant larvae protein homolog 1",
  "term_id": "GO:0032878",
  "term_label": "regulation of establishment or maintenance of cell polarity",
  "gene": "UniProtKB:Q15334"
}